{
  "term_id": "GO:0016018",
  "gene_name": "Peptidyl-prolyl cis-trans isomerase A-like 4D",
  "term_label": "cyclosporin A binding",
  "gene": "UniProtKB:F5H284",
  "gene_symbol": "PPIAL4D"
}